{
  "term_label": "Unknown cellular component",
  "term_id": "UNKNOWN:0003",
  "gene_symbol": "RTL8A",
  "gene_name": "Retrotransposon Gag-like protein 8A",
  "gene": "UniProtKB:Q9BWD3"
}